{
  "gene_symbol": "P2RY11",
  "term_label": "G protein-coupled receptor signaling pathway",
  "gene_name": "P2Y purinoceptor 11",
  "term_id": "GO:0007186",
  "gene": "UniProtKB:Q96G91"
}